{
  "term_label": "high voltage-gated calcium channel activity",
  "term_id": "GO:0008331",
  "gene_symbol": "CACNA1B",
  "gene_name": "Voltage-dependent N-type calcium channel subunit alpha-1B",
  "gene": "UniProtKB:Q00975"
}